{
  "gene_symbol": "HOXC10",
  "term_id": "GO:0005634",
  "term_label": "nucleus",
  "gene_name": "Homeobox protein Hox-C10",
  "gene": "UniProtKB:Q9NYD6"
}